phosphatidylglycerol alanyltransferase activity [GO:0047637] (molecular function) Also known as: alanyl phosphatidylglycerol synthetase activity Relationships: is a type of aminoacyltransferase activity [GO:0016755] Sources: EC:2.3.2.11 Definition: Catalysis of the reaction: 1,2-diacyl-sn-glycero-3-phospho-(1'-sn-glycerol) + L-alanyl-tRNA(Ala) = 1,2-diacyl-sn-glycero-3-phospho-1'-(3'-O-L-alanyl)-sn-glycerol + tRNA(Ala).